{
  "gene": "UniProtKB:P13686",
  "term_id": "UNKNOWN:0003",
  "term_label": "Unknown cellular component",
  "gene_symbol": "ACP5",
  "gene_name": "Tartrate-resistant acid phosphatase type 5"
}